contractile vacuole discharge [GO:0070177] (biological process) References: PMID:10369671 Sources: GOC:mah Definition: The regulated release of water from a contractile vacuole to the outside of a cell by fusion of the contractile vacuole membrane with the plasma membrane. Relationships: is a type of regulated exocytosis [GO:0045055]